response to prostaglandin F [GO:0034696] (biological process) Definition: Any process that results in a change in state or activity of a cell or an organism (in terms of movement, secretion, enzyme production, gene expression, etc.) as a result of a prostagladin F stimulus. Sources: GOC:BHF, GOC:vk Also known as: response to prostaglandin F stimulus Relationships: is a type of response to prostaglandin [GO:0034694] Subtypes: GO:0071381